{
  "term_id": "UNKNOWN:0002",
  "gene": "UniProtKB:Q8N6N6",
  "gene_name": "Protein NATD1",
  "gene_symbol": "NATD1",
  "term_label": "Unknown biological process"
}